{
  "term_label": "Unknown biological process",
  "gene": "UniProtKB:Q76KP1",
  "term_id": "UNKNOWN:0002",
  "gene_name": "N-acetyl-beta-glucosaminyl-glycoprotein 4-beta-N-acetylgalactosaminyltransferase 1",
  "gene_symbol": "B4GALNT4"
}